{
  "term_id": "UNKNOWN:0003",
  "gene_symbol": "A0A804HID5",
  "gene": "UniProtKB:A0A804HID5",
  "gene_name": "Uncharacterized protein",
  "term_label": "Unknown cellular component"
}